magnesium:sodium antiporter activity [GO:0061768] (molecular function) Relationships: is a type of GO:0015081; is a type of GO:0015095; is a type of GO:0140828 Definition: Catalysis of the reaction: Na+(in) + Mg2+(out) = Na+(out) + Mg2+(in). References: PMID:22031603 Sources: GOC:PARL, GOC:pad